ciliary basal body-plasma membrane docking [GO:0097711] (biological process) Definition: The docking of a cytosolic centriole/basal body to the plasma membrane via the ciliary transition fibers. In some species this may happen via an intermediate step, by first docking to the ciliary vesicle via the ciliary transition fibers. The basal body-ciliary vesicle then relocates to the plasma membrane, followed by the ciliary vesicle fusing with the plasma membrane, effectively attaching the basal body to the plasma membrane. References: PMID:13978319, PMID:23348840, PMID:23530209, PMID:25686250, PMID:26981235 Sources: GOC:cilia Also known as: ciliary basal body docking, anchoring of the basal body to the plasma membrane Note: Basal bodies in jawed vertebrates appear to first attach to a ciliary vesicle. It is unclear how specific this is to jawed vertebrates or if other organisms also employ this sequence. Some species like Giardia intestinalis do not relocate their basal bodies to the plasma membrane, but have their axonemes extend through the cytosol to then protrude out of the cell to form flagella. Relationships: is a type of organelle localization by membrane tethering [GO:0140056]; BFO_0000050 GO:0060271